{
  "term_label": "extracellular space",
  "gene_name": "Protein Wnt-6",
  "gene": "UniProtKB:Q9Y6F9",
  "gene_symbol": "WNT6",
  "term_id": "GO:0005615"
}